{
  "term_id": "UNKNOWN:0001",
  "gene": "UniProtKB:Q3KRA9",
  "gene_symbol": "ALKBH6",
  "term_label": "Unknown molecular function",
  "gene_name": "Alpha-ketoglutarate-dependent dioxygenase alkB homolog 6"
}